pronephric duct development [GO:0039022] (biological process) Definition: The process whose specific outcome is the progression of the pronephric duct over time, from its formation to the mature structure. The pronephric duct collects the filtrate from the pronephric tubules and opens to the exterior of the pronephric kidney. References: PMID:15647339 Sources: GOC:mtg_kidney_jan10, XAO:0000063, ZFA:0000150 Relationships: is a type of nephric duct development [GO:0072176]; is part of pronephros development [GO:0048793]